{
  "gene_symbol": "MED12",
  "term_id": "GO:0045944",
  "gene_name": "Mediator of RNA polymerase II transcription subunit 12",
  "gene": "UniProtKB:Q93074",
  "term_label": "positive regulation of transcription by RNA polymerase II"
}